{
  "gene_symbol": "CPSF4",
  "gene": "UniProtKB:O95639",
  "term_label": "Unknown molecular function",
  "term_id": "UNKNOWN:0001",
  "gene_name": "Cleavage and polyadenylation specificity factor subunit 4"
}